{
  "term_label": "ubiquitin conjugating enzyme binding",
  "gene_name": "E3 ubiquitin-protein ligase SIAH2",
  "gene": "UniProtKB:O43255",
  "term_id": "GO:0031624",
  "gene_symbol": "SIAH2"
}